{
  "gene_symbol": "Q6ZS49",
  "term_label": "Unknown cellular component",
  "term_id": "UNKNOWN:0003",
  "gene_name": "Putative uncharacterized protein FLJ45831",
  "gene": "UniProtKB:Q6ZS49"
}